{
  "term_id": "UNKNOWN:0003",
  "term_label": "Unknown cellular component",
  "gene": "UniProtKB:Q5XKR4",
  "gene_name": "Homeobox protein orthopedia",
  "gene_symbol": "OTP"
}